{
  "gene_symbol": "RPL4",
  "term_id": "GO:0003735",
  "gene": "UniProtKB:P36578",
  "term_label": "structural constituent of ribosome",
  "gene_name": "Large ribosomal subunit protein uL4"
}